{
  "gene_symbol": "TMED3",
  "gene_name": "Transmembrane emp24 domain-containing protein 3",
  "term_label": "Unknown molecular function",
  "term_id": "UNKNOWN:0001",
  "gene": "UniProtKB:Q9Y3Q3"
}